{
  "gene_symbol": "MYH2",
  "gene": "UniProtKB:Q9UKX2",
  "term_id": "GO:0005737",
  "gene_name": "Myosin-2",
  "term_label": "cytoplasm"
}